{
  "gene_name": "Protein disulfide-isomerase A4",
  "gene": "UniProtKB:P13667",
  "term_label": "response to endoplasmic reticulum stress",
  "term_id": "GO:0034976",
  "gene_symbol": "PDIA4"
}